vesicle-mediated transport [GO:0016192] (BP) Subtypes: exocytosis [GO:0006887], GO:0006897, GO:0008333, endosomal transport [GO:0016197], retrograde transport, plasma membrane to Golgi [GO:0035526], transcytosis [GO:0045056], late endosome to vacuole transport [GO:0045324], Golgi vesicle transport [GO:0048193], GO:0048227, multivesicular body sorting pathway [GO:0071985], vesicle-mediated cholesterol transport [GO:0090119], lysosome to ER cholesterol transport [GO:0090120], vesicle-mediated transport to the plasma membrane [GO:0098876], GO:0098968, vesicle-mediated transport in synapse [GO:0099003], mitochondrion-derived vesicle mediated transport [GO:0099075], vesicle-mediated intercellular transport [GO:0110077], GO:0140026, plastid to vacuole vesicle-mediated transport [GO:1904962] Definition: A cellular transport process in which transported substances are moved in membrane-bounded vesicles; transported substances are enclosed in the vesicle lumen or located in the vesicle membrane. The process begins with a step that directs a substance to the forming vesicle, and includes vesicle budding and coating. Vesicles are then targeted to, and fuse with, an acceptor membrane. Also known as: vesicle transport, vesicular transport, nonselective vesicle transport, protein sorting along secretory pathway, vesicle trafficking Sources: GOC:ai, GOC:mah, ISBN:08789310662000 Regulation: regulated by regulation of vesicle-mediated transport [GO:0060627] Relationships: is a type of GO:0006810; is a type of GO:0009987